{
  "gene": "UniProtKB:Q3ZCN5",
  "gene_symbol": "OTOGL",
  "term_id": "GO:0005201",
  "term_label": "extracellular matrix structural constituent",
  "gene_name": "Otogelin-like protein"
}